positive regulation of type II interferon-mediated signaling pathway [GO:0060335] (biological process) Relationships: is a type of positive regulation of cytokine-mediated signaling pathway [GO:0001961]; is a type of positive regulation of response to type II interferon [GO:0060332]; is a type of GO:0060334; positively regulates type II interferon-mediated signaling pathway [GO:0060333] Also known as: positive regulation of interferon-gamma-mediated signaling pathway, positive regulation of type II IFN-mediated pathway, positive regulation of immune interferon-mediated signaling pathway, positive regulation of interferon-gamma-mediated signalling pathway, positive regulation of gamma-interferon-mediated signaling pathway Sources: GOC:dph Definition: Any process that increases the rate, frequency or extent of an interferon-gamma-mediated signaling pathway.